{
  "gene_symbol": "PYCARD",
  "term_id": "GO:0038187",
  "gene_name": "Apoptosis-associated speck-like protein containing a CARD",
  "term_label": "pattern recognition receptor activity",
  "gene": "UniProtKB:Q9ULZ3"
}